CoA carboxylase activity [GO:0016421] (molecular function) Definition: Catalysis of the joining of a carboxyl group to a molecule that is attached to CoA, with the concomitant hydrolysis of the diphosphate bond in ATP or a similar triphosphate. Sources: GOC:mah Relationships: is a type of ligase activity, forming carbon-carbon bonds [GO:0016885] Subtypes: GO:0003989, methylcrotonoyl-CoA carboxylase activity [GO:0004485], GO:0004658, geranoyl-CoA carboxylase activity [GO:0047925]